{
  "gene_name": "Hemoglobin subunit zeta",
  "term_id": "GO:0020037",
  "term_label": "heme binding",
  "gene_symbol": "HBZ",
  "gene": "UniProtKB:P02008"
}